{
  "gene": "UniProtKB:Q9UII2",
  "term_label": "ATPase inhibitor activity",
  "term_id": "GO:0042030",
  "gene_symbol": "ATP5IF1",
  "gene_name": "ATPase inhibitor, mitochondrial"
}